elongator holoenzyme complex [GO:0033588] (cellular component) Definition: A heterohexameric protein complex composed two discrete heterotrimeric subcomplexes that is involved in modification of wobble nucleosides in tRNA. References: PMID:11435442, PMID:11689709, PMID:15769872, PMID:17018299, PMID:18755837, PMID:23165209 Sources: GOC:bhm, GOC:jh, GOC:mah, GOC:vw Also known as: Elongator core complex Note: Despite its name, this complex is not directly involved in transcriptional elongation (PMID:23165209). Relationships: is a type of intracellular protein-containing complex [GO:0140535]; is a type of catalytic complex [GO:1902494]